{
  "gene_name": "Potassium_sodium hyperpolarization-activated cyclic nucleotide-gated channel 3",
  "term_label": "regulation of membrane depolarization",
  "gene": "UniProtKB:Q9P1Z3",
  "term_id": "GO:0003254",
  "gene_symbol": "HCN3"
}